microgametophyte vegetative cell differentiation [GO:0022620] (biological process) Also known as: tube cell differentiation, vegetative cell differentiation Sources: GOC:isa_complete Relationships: is a type of cell differentiation [GO:0030154]; is part of microgametogenesis [GO:0055046] Definition: The process in which a relatively unspecialized cell acquires specialized features of a microgametophyte. The microgametophyte vegetative cell gives rise to the pollen tube.